{
  "term_label": "mitochondrial membrane",
  "gene_name": "Interferon alpha-inducible protein 27-like protein 1",
  "gene": "UniProtKB:Q96BM0",
  "gene_symbol": "IFI27L1",
  "term_id": "GO:0031966"
}